protein kinase B binding [GO:0043422] (molecular function) Relationships: is a type of GO:0019901 Definition: Binding to protein kinase B, an intracellular kinase that is important in regulating glucose metabolism. Also known as: Akt binding, PKB binding Sources: GOC:jl, https://doi.org/10.1016/S0092-8674(02)01083-8